{
  "gene": "UniProtKB:Q8NGC4",
  "term_label": "olfactory receptor activity",
  "gene_name": "Olfactory receptor 10G3",
  "gene_symbol": "OR10G3",
  "term_id": "GO:0004984"
}